regulation of mitotic chromosome condensation [GO:1903379] (biological process) Definition: Any process that modulates the frequency, rate or extent of mitotic chromosome condensation. References: PMID:9490640 Sources: GOC:TermGenie, GO_REF:0000058 Relationships: is a type of regulation of cell cycle process [GO:0010564]; is a type of regulation of chromosome condensation [GO:0060623]; regulates mitotic chromosome condensation [GO:0007076] Subtypes: GO:1903380, negative regulation of mitotic chromosome condensation [GO:1905213]